{
  "term_id": "UNKNOWN:0003",
  "gene_symbol": "FAM184A",
  "gene_name": "Protein FAM184A",
  "gene": "UniProtKB:Q8NB25",
  "term_label": "Unknown cellular component"
}